glycoprotein biosynthetic process [GO:0009101] (biological process) Definition: The chemical reactions and pathways resulting in the formation of glycoproteins, a protein that contains covalently bound glycose (i.e. monosaccharide) residues; the glycose occurs most commonly as oligosaccharide or fairly small polysaccharide but occasionally as monosaccharide. References: PMID:35536965 Also known as: glycoprotein anabolism, glycoprotein biosynthesis, glycoprotein formation, glycoprotein synthesis Relationships: is a type of GO:0009059; is a type of glycoprotein metabolic process [GO:0009100]; is a type of carbohydrate derivative biosynthetic process [GO:1901137] Subtypes: GO:0006487, GO:0006491, GO:0006493, protein C-linked glycosylation [GO:0018103], protein S-linked glycosylation [GO:0018280], proteoglycan biosynthetic process [GO:0030166], cell wall glycoprotein biosynthetic process [GO:0031506], protein phosphate-linked glycosylation [GO:0042076], protein post-translational transfer of dolichol-linked oligosaccharide [GO:0180057], GO:0180058 Regulation: regulated by regulation of glycoprotein biosynthetic process [GO:0010559]; positively regulated by positive regulation of glycoprotein biosynthetic process [GO:0010560]; negatively regulated by negative regulation of glycoprotein biosynthetic process [GO:0010561]